{
  "term_id": "GO:0007032",
  "gene": "UniProtKB:Q9Y6D5",
  "gene_name": "Brefeldin A-inhibited guanine nucleotide-exchange protein 2",
  "term_label": "endosome organization",
  "gene_symbol": "ARFGEF2"
}